positive regulation of direction of cell growth [GO:0061390] (biological process) Sources: GOC:mah, GOC:vw Definition: Any process that increases the direction of cell growth. Relationships: is a type of GO:0030307; is a type of regulation of direction of cell growth [GO:0061389]